{
  "term_label": "Unknown biological process",
  "term_id": "UNKNOWN:0002",
  "gene": "UniProtKB:Q8NEL0",
  "gene_symbol": "CCDC54",
  "gene_name": "Coiled-coil domain-containing protein 54"
}